{
  "gene_name": "Pre-mRNA-splicing factor SYF1",
  "gene_symbol": "XAB2",
  "gene": "UniProtKB:Q9HCS7",
  "term_label": "mRNA splicing, via spliceosome",
  "term_id": "GO:0000398"
}